{
  "gene_name": "Protein arginine N-methyltransferase 8",
  "term_id": "GO:0035242",
  "gene_symbol": "PRMT8",
  "term_label": "protein-arginine omega-N asymmetric methyltransferase activity",
  "gene": "UniProtKB:Q9NR22"
}